{
  "term_label": "Unknown cellular component",
  "term_id": "UNKNOWN:0003",
  "gene": "UniProtKB:Q9NUL5",
  "gene_name": "Shiftless antiviral inhibitor of ribosomal frameshifting protein",
  "gene_symbol": "SHFL"
}